{
  "term_label": "focal adhesion",
  "term_id": "GO:0005925",
  "gene_symbol": "DST",
  "gene_name": "Dystonin",
  "gene": "UniProtKB:Q03001"
}